{
  "term_label": "nucleus",
  "gene_name": "Regulator of G-protein signaling 3",
  "gene_symbol": "RGS3",
  "term_id": "GO:0005634",
  "gene": "UniProtKB:P49796"
}